{
  "gene_name": "Protein SERAC1",
  "gene": "UniProtKB:Q96JX3",
  "gene_symbol": "SERAC1",
  "term_label": "phosphatidylglycerol acyl-chain remodeling",
  "term_id": "GO:0036148"
}